trimethylenediamine biosynthetic process [GO:1901057] (biological process) Definition: The chemical reactions and pathways resulting in the formation of trimethylenediamine. Sources: GOC:TermGenie, GOC:yaf, UniPathway:UPA00010 Also known as: trimethylenediamine anabolism, trimethylenediamine biosynthesis, trimethylenediamine formation, trimethylenediamine synthesis Relationships: is a type of polyamine biosynthetic process [GO:0006596]